{
  "term_label": "heme binding",
  "gene_symbol": "HMOX2",
  "gene_name": "Heme oxygenase 2",
  "term_id": "GO:0020037",
  "gene": "UniProtKB:P30519"
}